{
  "term_label": "Unknown molecular function",
  "gene_name": "Coiled-coil domain-containing protein 120",
  "term_id": "UNKNOWN:0001",
  "gene": "UniProtKB:Q96HB5",
  "gene_symbol": "CCDC120"
}